{
  "term_id": "GO:0010468",
  "gene_name": "Activity-dependent neuroprotector homeobox protein",
  "term_label": "regulation of gene expression",
  "gene_symbol": "ADNP",
  "gene": "UniProtKB:Q9H2P0"
}